{
  "gene_name": "Dihydropyrimidinase-related protein 2",
  "gene_symbol": "DPYSL2",
  "gene": "UniProtKB:Q16555",
  "term_id": "GO:0016812",
  "term_label": "hydrolase activity, acting on carbon-nitrogen (but not peptide) bonds, in cyclic amides"
}